{
  "term_id": "GO:0000724",
  "term_label": "double-strand break repair via homologous recombination",
  "gene_name": "Structural maintenance of chromosomes protein 5",
  "gene": "UniProtKB:Q8IY18",
  "gene_symbol": "SMC5"
}